{
  "term_label": "aldehyde metabolic process",
  "gene_symbol": "ALDH1A1",
  "gene_name": "Aldehyde dehydrogenase 1A1",
  "gene": "UniProtKB:P00352",
  "term_id": "GO:0006081"
}